{
  "term_label": "nucleus",
  "gene_symbol": "DYRK2",
  "term_id": "GO:0005634",
  "gene": "UniProtKB:Q92630",
  "gene_name": "Dual specificity tyrosine-phosphorylation-regulated kinase 2"
}